extracellular negative regulation of signal transduction [GO:1900116] (biological process) Relationships: is a type of negative regulation of signal transduction [GO:0009968]; is a type of GO:1900115 Sources: GOC:TermGenie, GOC:signaling Definition: Any negative regulation of signal transduction that takes place in extracellular region. Subtypes: sequestering of extracellular ligand from receptor [GO:0035581] Also known as: down regulation of signal transduction in extracellular region, down-regulation of signal transduction in extracellular region, downregulation of signal transduction in extracellular region, negative regulation of signaling pathway in extracellular region, negative regulation of signalling pathway in extracellular region, extracellular inhibition of signaling pathway, inhibition of signal transduction in extracellular region